{
  "gene": "UniProtKB:Q8TEU8",
  "gene_symbol": "WFIKKN2",
  "term_label": "transforming growth factor beta receptor signaling pathway",
  "gene_name": "WAP, Kazal, immunoglobulin, Kunitz and NTR domain-containing protein 2",
  "term_id": "GO:0007179"
}